{
  "gene_symbol": "CCT8",
  "gene_name": "T-complex protein 1 subunit theta",
  "term_label": "unfolded protein binding",
  "gene": "UniProtKB:P50990",
  "term_id": "GO:0051082"
}